{
  "gene_name": "Threonine synthase-like 2",
  "gene": "UniProtKB:Q86YJ6",
  "gene_symbol": "THNSL2",
  "term_label": "Unknown biological process",
  "term_id": "UNKNOWN:0002"
}